{
  "term_label": "Unknown biological process",
  "gene_symbol": "LONRF1",
  "gene_name": "LON peptidase N-terminal domain and RING finger protein 1",
  "gene": "UniProtKB:Q17RB8",
  "term_id": "UNKNOWN:0002"
}